{
  "term_id": "UNKNOWN:0002",
  "term_label": "Unknown biological process",
  "gene_name": "Small integral membrane protein 19",
  "gene": "UniProtKB:Q96E16",
  "gene_symbol": "SMIM19"
}